response to psychosocial stress [GO:1990911] (biological process) Relationships: is a type of GO:0006950 Definition: Any process that results in a change in state or activity of a cell or an organism (in terms of movement, secretion, enzyme production, gene expression, etc.) as a result of exposure to aversive or demanding psychological and social conditions that tax or exceed the behavioral resources of the organism. References: PMID:22922217, PMID:26458179